type 4 melanocortin receptor binding [GO:0031782] (molecular function) Also known as: type 4 melanocortin receptor ligand Definition: Binding to a type 4 melanocortin receptor. Relationships: is a type of melanocortin receptor binding [GO:0031779] Sources: GOC:mah, GOC:nln